{
  "term_label": "DNA binding",
  "gene_symbol": "BCLAF3",
  "gene": "UniProtKB:A2AJT9",
  "gene_name": "BCLAF1 and THRAP3 family member 3",
  "term_id": "GO:0003677"
}